{
  "term_id": "UNKNOWN:0003",
  "gene_symbol": "CRCT1",
  "term_label": "Unknown cellular component",
  "gene": "UniProtKB:Q9UGL9",
  "gene_name": "Cysteine-rich C-terminal protein 1"
}